{
  "gene": "UniProtKB:Q6UWI2",
  "gene_name": "Prostate androgen-regulated mucin-like protein 1",
  "term_label": "Unknown molecular function",
  "gene_symbol": "PARM1",
  "term_id": "UNKNOWN:0001"
}